{
  "term_label": "Unknown biological process",
  "term_id": "UNKNOWN:0002",
  "gene_symbol": "AKR1E2",
  "gene_name": "1,5-anhydro-D-fructose reductase",
  "gene": "UniProtKB:Q96JD6"
}